{
  "term_label": "DNA-binding transcription factor activity",
  "gene_symbol": "POGZ",
  "gene": "UniProtKB:Q7Z3K3",
  "term_id": "GO:0003700",
  "gene_name": "Pogo transposable element with ZNF domain"
}